{
  "gene": "UniProtKB:O95402",
  "term_id": "GO:0010628",
  "term_label": "positive regulation of gene expression",
  "gene_name": "Mediator of RNA polymerase II transcription subunit 26",
  "gene_symbol": "MED26"
}